{
  "term_id": "UNKNOWN:0001",
  "gene_name": "Membrane-anchored junction protein",
  "gene": "UniProtKB:Q3KP22",
  "gene_symbol": "MAJIN",
  "term_label": "Unknown molecular function"
}